diguanidinobutanase activity [GO:0047854] (molecular function) Definition: Catalysis of the reaction: 1,4-diguanidinobutane + H2O = agmatine + urea. Relationships: is a type of hydrolase activity, acting on carbon-nitrogen (but not peptide) bonds, in linear amidines [GO:0016813] Also known as: 1,4-diguanidinobutane amidinohydrolase activity Sources: EC:3.5.3.20, RHEA:13597